{
  "gene": "UniProtKB:Q9NXH9",
  "term_id": "GO:0160104",
  "gene_name": "tRNA (guanine(26)-N(2))-dimethyltransferase",
  "gene_symbol": "TRMT1",
  "term_label": "tRNA (guanine(26)-N2)-dimethyltransferase activity"
}